{
  "gene": "UniProtKB:Q02297",
  "term_label": "brain development",
  "gene_symbol": "NRG1",
  "gene_name": "Pro-neuregulin-1, membrane-bound isoform",
  "term_id": "GO:0007420"
}